{
  "gene": "UniProtKB:Q9BUJ2",
  "gene_symbol": "HNRNPUL1",
  "gene_name": "Heterogeneous nuclear ribonucleoprotein U-like protein 1",
  "term_label": "nucleus",
  "term_id": "GO:0005634"
}